guaiacyl lignin biosynthetic process [GO:1901063] (biological process) Sources: GOC:TermGenie, GOC:mengo_curators Relationships: is a type of lignin biosynthetic process [GO:0009809] Definition: The chemical reactions and pathways resulting in the formation of guaiacyl lignin. Also known as: G-lignin biosynthetic process, guaiacyl lignin anabolism, guaiacyl lignin biosynthesis, guaiacyl lignin formation, guaiacyl lignin synthesis